symbiont-mediated suppression of host peptidoglycan biosynthetic process [GO:0039635] (biological process) Definition: Any process in which a symbiont stops, prevents, or reduces the frequency, rate or extent of peptidoglycan biosynthesis in the host organism. Peptidoglycans are any of a class of glycoconjugates found in bacterial cell walls, and phages have mechanisms to disrupt their host's cell walls. Relationships: is a type of symbiont-mediated perturbation of host cellular process [GO:0044068] Sources: GOC:bf, GOC:bm, GOC:jl Also known as: suppression by virus of host peptidoglycan biosynthetic process, viral inhibition of host peptidoglycan biosynthesis